{
  "term_label": "nucleus",
  "gene": "UniProtKB:P42772",
  "gene_symbol": "CDKN2B",
  "gene_name": "Cyclin-dependent kinase 4 inhibitor B",
  "term_id": "GO:0005634"
}